{
  "gene": "UniProtKB:Q7Z589",
  "gene_symbol": "EMSY",
  "term_label": "Unknown molecular function",
  "term_id": "UNKNOWN:0001",
  "gene_name": "BRCA2-interacting transcriptional repressor EMSY"
}